{
  "term_label": "microtubule binding",
  "term_id": "GO:0008017",
  "gene_name": "Cytoskeleton-associated protein 5",
  "gene_symbol": "CKAP5",
  "gene": "UniProtKB:Q14008"
}